{
  "gene_name": "Eukaryotic translation initiation factor 3 subunit G",
  "term_label": "eukaryotic translation initiation factor 3 complex",
  "term_id": "GO:0005852",
  "gene_symbol": "EIF3G",
  "gene": "UniProtKB:O75821"
}